{
  "gene": "UniProtKB:B2RU33",
  "gene_name": "POTE ankyrin domain family member C",
  "term_id": "UNKNOWN:0002",
  "term_label": "Unknown biological process",
  "gene_symbol": "POTEC"
}